phosphoenolpyruvate phosphatase activity [GO:0050189] (molecular function) Relationships: is a type of phosphatase activity [GO:0016791] Definition: Catalysis of the reaction: H2O + phosphoenolpyruvate = phosphate + pyruvate. Sources: EC:3.1.3.60, RHEA:19997 Also known as: PEP phosphatase activity, phosphoenolpyruvate phosphohydrolase activity